{
  "term_id": "GO:0005886",
  "term_label": "plasma membrane",
  "gene_name": "Killer cell immunoglobulin-like receptor 2DS1",
  "gene": "UniProtKB:Q14954",
  "gene_symbol": "KIR2DS1"
}